{
  "gene_name": "Isochorismatase domain-containing protein 2",
  "gene_symbol": "ISOC2",
  "gene": "UniProtKB:Q96AB3",
  "term_label": "Unknown molecular function",
  "term_id": "UNKNOWN:0001"
}